response to histamine [GO:0034776] (biological process) Definition: Any process that results in a change in state or activity of a cell or an organism (in terms of movement, secretion, enzyme production, gene expression, etc.) as a result of a histamine stimulus. Histamine, the biogenic amine 2-(1H-imidazol-4-yl)ethanamine, is involved in local immune responses as well as regulating physiological function in the gut and acting as a neurotransmitter. Relationships: is a type of response to nitrogen compound [GO:1901698] Sources: GOC:BHF, GOC:mah, GOC:vk Also known as: response to histamine stimulus Subtypes: cellular response to histamine [GO:0071420], GO:0097280